immunoglobulin complex, circulating [GO:0042571] (cellular component) Relationships: is a type of GO:0019814; is part of extracellular space [GO:0005615] Definition: An immunoglobulin complex that is secreted into extracellular space and found in mucosal areas or other tissues or circulating in the blood or lymph. In its canonical form, a circulating immunoglobulin complex is composed of two identical heavy chains and two identical light chains, held together by disulfide bonds. Some forms of are polymers of the basic structure and contain additional components such as J-chain and the secretory component. Sources: GOC:add, ISBN:0781735149 Note: Note that an immunoglobulin complex has the function of antigen binding if a suitable antigen is available. Also known as: antibody Subtypes: IgG immunoglobulin complex, circulating [GO:0071736], IgD immunoglobulin complex, circulating [GO:0071739], IgE immunoglobulin complex, circulating [GO:0071743], IgA immunoglobulin complex, circulating [GO:0071746], GO:0071754